{
  "term_id": "UNKNOWN:0002",
  "term_label": "Unknown biological process",
  "gene": "UniProtKB:O96007",
  "gene_symbol": "MOCS2",
  "gene_name": "Molybdopterin synthase catalytic subunit"
}